calcium ion transmembrane transport [GO:0070588] (biological process) Note: Note that this term is not intended for use in annotating lateral movement within membranes. Relationships: is a type of calcium ion transport [GO:0006816]; is a type of monoatomic cation transmembrane transport [GO:0098655] Also known as: calcium ion membrane transport, transmembrane calcium transport Sources: GOC:mah Subtypes: GO:0006851, calcium ion transmembrane transport via high voltage-gated calcium channel [GO:0061577], Golgi calcium ion transmembrane transport [GO:0061856], calcium ion transmembrane transport via low voltage-gated calcium channel [GO:0090676], calcium ion transmembrane import into cytosol [GO:0097553], GO:0140146, GO:1903515, calcium ion export across plasma membrane [GO:1990034] Definition: A process in which a calcium ion is transported from one side of a membrane to the other by means of some agent such as a transporter or pore. Regulation: regulated by regulation of calcium ion transmembrane transport [GO:1903169]; negatively regulated by negative regulation of calcium ion transmembrane transport [GO:1903170]; positively regulated by positive regulation of calcium ion transmembrane transport [GO:1904427]